N-methyl-L-amino-acid oxidase activity [GO:0050131] (molecular function) Definition: Catalysis of the reaction: an N-methyl-L-amino acid + H2O + O2 = an L-amino acid + formaldehyde + H2O2. Relationships: is a type of oxidoreductase activity, acting on the CH-NH group of donors, oxygen as acceptor [GO:0016647] Also known as: N-methyl-L-amino-acid:oxygen oxidoreductase (demethylating), N-methylamino acid oxidase activity Sources: EC:1.5.3.2